regulation of receptor-mediated endocytosis [GO:0048259] (biological process) Relationships: is a type of regulation of endocytosis [GO:0030100]; regulates receptor-mediated endocytosis [GO:0006898] Also known as: regulation of receptor mediated endocytosis Subtypes: GO:0002090, positive regulation of receptor-mediated endocytosis [GO:0048260], negative regulation of receptor-mediated endocytosis [GO:0048261], regulation of receptor-mediated endocytosis involved in cholesterol transport [GO:1905600], regulation of clathrin-dependent endocytosis [GO:2000369] Definition: Any process that modulates the frequency, rate or extent of receptor mediated endocytosis, the uptake of external materials by cells, utilizing receptors to ensure specificity of transport. Sources: GOC:go_curators, GOC:tb